{
  "gene": "UniProtKB:A1L170",
  "term_label": "Unknown biological process",
  "gene_name": "Uncharacterized protein C1orf226",
  "term_id": "UNKNOWN:0002",
  "gene_symbol": "C1orf226"
}